lactate 2-monooxygenase activity [GO:0050040] (molecular function) Relationships: is a type of oxidoreductase activity, acting on single donors with incorporation of molecular oxygen, incorporation of one atom of oxygen (internal monooxygenases or internal mixed function oxidases) [GO:0016703] Sources: EC:1.13.12.4, RHEA:16513 Definition: Catalysis of the reaction: (S)-lactate + O2 = acetate + CO2 + H2O. Also known as: (S)-lactate:oxygen 2-oxidoreductase (decarboxylating), L-lactate monooxygenase activity, L-lactate-2-monooxygenase activity, lactate monooxygenase activity, lactate oxidase activity, lactate oxidative decarboxylase activity, lactate oxygenase activity, lactic oxidase activity, lactic oxygenase activity